regulation of respiratory gaseous exchange [GO:0043576] (biological process) Definition: Any process that modulates the frequency, rate or extent of the process of gaseous exchange between an organism and its environment. Sources: GOC:jl Relationships: is a type of regulation of multicellular organismal process [GO:0051239]; regulates respiratory gaseous exchange by respiratory system [GO:0007585] Subtypes: regulation of respiratory system process [GO:0044065], negative regulation of respiratory gaseous exchange [GO:1903941], positive regulation of respiratory gaseous exchange [GO:1903942]